{
  "gene_name": "Sonic hedgehog protein",
  "gene_symbol": "SHH",
  "term_id": "GO:0001708",
  "gene": "UniProtKB:Q15465",
  "term_label": "cell fate specification"
}